{
  "gene": "UniProtKB:Q96KR1",
  "gene_name": "Zinc finger RNA-binding protein",
  "gene_symbol": "ZFR",
  "term_id": "GO:0003727",
  "term_label": "single-stranded RNA binding"
}